{
  "gene": "UniProtKB:P05106",
  "gene_symbol": "ITGB3",
  "term_label": "integrin-mediated signaling pathway",
  "gene_name": "Integrin beta-3",
  "term_id": "GO:0007229"
}